{
  "term_label": "Golgi organization",
  "gene_name": "Transmembrane emp24 domain-containing protein 6",
  "gene_symbol": "TMED6",
  "gene": "UniProtKB:Q8WW62",
  "term_id": "GO:0007030"
}